{
  "gene_name": "Bile salt-activated lipase",
  "gene_symbol": "CEL",
  "gene": "UniProtKB:P19835",
  "term_id": "GO:0004806",
  "term_label": "triacylglycerol lipase activity"
}